thiosulfate dehydrogenase (quinone) activity [GO:0043831] (molecular function) Relationships: is a type of oxidoreductase activity, acting on a sulfur group of donors, quinone or similar compound as acceptor [GO:0016672] Also known as: thiosulphate dehydrogenase (quinone) activity, thiosulphate:quinone oxidoreductase activity, DoxA, DoxD, TQO, thiosulfate oxidoreductase, tetrathionate-forming activity, thiosulfate:6-decylubiquinone oxidoreductase activity, thiosulfate:quinone oxidoreductase activity Definition: Catalysis of the reaction: 6-decylubiquinone + 2 thiosulfate = 6-decylubiquinol + tetrathionate. Sources: RHEA:10936